{
  "gene_name": "Kallikrein-1",
  "term_label": "extracellular space",
  "term_id": "GO:0005615",
  "gene": "UniProtKB:P06870",
  "gene_symbol": "KLK1"
}